{
  "term_id": "GO:0005109",
  "term_label": "frizzled binding",
  "gene_symbol": "WNT10B",
  "gene": "UniProtKB:O00744",
  "gene_name": "Protein Wnt-10b"
}